{
  "term_id": "GO:0043401",
  "gene_name": "Monoacylglycerol lipase ABHD2",
  "term_label": "steroid hormone receptor signaling pathway",
  "gene": "UniProtKB:P08910",
  "gene_symbol": "ABHD2"
}